{
  "gene_symbol": "HIBCH",
  "gene": "UniProtKB:Q6NVY1",
  "term_id": "GO:0006574",
  "term_label": "L-valine catabolic process",
  "gene_name": "3-hydroxyisobutyryl-CoA hydrolase, mitochondrial"
}